{
  "gene_symbol": "ANKS6",
  "gene": "UniProtKB:Q68DC2",
  "term_label": "cytoplasm",
  "gene_name": "Ankyrin repeat and SAM domain-containing protein 6",
  "term_id": "GO:0005737"
}